{
  "term_label": "lipid transporter activity",
  "gene_name": "Phospholipid-transporting ATPase ABCA3",
  "gene_symbol": "ABCA3",
  "gene": "UniProtKB:Q99758",
  "term_id": "GO:0005319"
}